{
  "gene_name": "G-protein coupled receptor 22",
  "term_label": "G protein-coupled receptor signaling pathway",
  "term_id": "GO:0007186",
  "gene": "UniProtKB:Q99680",
  "gene_symbol": "GPR22"
}